{
  "term_label": "Unknown molecular function",
  "gene_symbol": "PSENEN",
  "gene": "UniProtKB:Q9NZ42",
  "term_id": "UNKNOWN:0001",
  "gene_name": "Gamma-secretase subunit PEN-2"
}